{
  "gene_name": "Protein ITPRID1",
  "gene_symbol": "ITPRID1",
  "term_label": "Unknown cellular component",
  "gene": "UniProtKB:Q6ZRS4",
  "term_id": "UNKNOWN:0003"
}